{
  "gene_name": "MAGUK p55 subfamily member 3",
  "gene": "UniProtKB:Q13368",
  "term_id": "UNKNOWN:0001",
  "term_label": "Unknown molecular function",
  "gene_symbol": "MPP3"
}